{
  "gene": "UniProtKB:Q2TAC6",
  "gene_name": "Kinesin-like protein KIF19",
  "term_label": "cytoplasm",
  "term_id": "GO:0005737",
  "gene_symbol": "KIF19"
}